{
  "gene_name": "Fascin",
  "term_id": "GO:0031253",
  "term_label": "cell projection membrane",
  "gene_symbol": "FSCN1",
  "gene": "UniProtKB:Q16658"
}